establishment of protein localization to telomere [GO:0070200] (biological process) Also known as: establishment of protein localisation to telomere, establishment of protein localization to chromosome, telomeric region Sources: GOC:BHF, GOC:mah Relationships: is a type of establishment of protein localization to chromosome [GO:0070199] Regulation: regulated by regulation of establishment of protein localization to telomere [GO:0070203]; negatively regulated by negative regulation of establishment of protein localization to telomere [GO:1904850]; positively regulated by positive regulation of establishment of protein localization to telomere [GO:1904851] Definition: The directed movement of a protein to a specific location in the telomeric region of a chromosome.